male courtship behavior, tapping to detect pheromone [GO:0016544] (biological process) Relationships: is a type of male courtship behavior [GO:0008049] References: PMID:11092827 Sources: GOC:mtg_sensu Also known as: male courtship behaviour, tapping, male courtship behavior, tapping, male courtship behaviour, tapping to detect pheromone Definition: The process during courtship where the male insect taps the female with his frontal leg. An example of this is found in Drosophila melanogaster.